{
  "term_label": "extracellular matrix",
  "gene_symbol": "RELN",
  "gene_name": "Reelin",
  "term_id": "GO:0031012",
  "gene": "UniProtKB:P78509"
}